{
  "term_label": "plasma membrane",
  "gene_name": "Metalloreductase STEAP1",
  "gene_symbol": "STEAP1",
  "gene": "UniProtKB:Q9UHE8",
  "term_id": "GO:0005886"
}